{
  "gene": "UniProtKB:Q8N300",
  "gene_symbol": "SVBP",
  "term_label": "Unknown molecular function",
  "gene_name": "Small vasohibin-binding protein",
  "term_id": "UNKNOWN:0001"
}